{
  "gene_name": "Importin subunit alpha-8",
  "term_label": "nuclear localization sequence binding",
  "gene": "UniProtKB:A9QM74",
  "term_id": "GO:0008139",
  "gene_symbol": "KPNA7"
}